{
  "term_id": "GO:0008284",
  "term_label": "positive regulation of cell population proliferation",
  "gene_name": "Proheparin-binding EGF-like growth factor",
  "gene": "UniProtKB:Q99075",
  "gene_symbol": "HBEGF"
}